taxadiene 5-alpha-hydroxylase activity [GO:0050604] (molecular function) Sources: RHEA:14049 Also known as: taxadiene 5a-hydroxylase activity, taxa-4,11-diene,hydrogen-donor:oxygen oxidoreductase (5alpha-hydroxylating), taxadiene 5alpha-hydroxylase activity Definition: Catalysis of the reaction: AH2 + O2 + taxa-4,11-diene = A + H2O + taxa-4(20),11-dien-5alpha-ol. Relationships: is a type of GO:0004497; is a type of oxidoreductase activity, acting on paired donors, with incorporation or reduction of molecular oxygen [GO:0016705]